positive regulation of response to cycloalkane [GO:1901433] (biological process) Sources: GOC:TermGenie, GOC:mengo_curators Also known as: up regulation of response to cycloalkane, up-regulation of response to cycloalkane, upregulation of response to cycloalkane, activation of response to cycloalkane Definition: Any process that activates or increases the frequency, rate or extent of response to cycloalkane. Relationships: is a type of positive regulation of response to stimulus [GO:0048584]; is a type of regulation of response to cycloalkane [GO:1901431]; positively regulates response to cycloalkane [GO:0014071]